{
  "gene_symbol": "ITM2B",
  "gene": "UniProtKB:Q9Y287",
  "gene_name": "Integral membrane protein 2B",
  "term_id": "GO:0005886",
  "term_label": "plasma membrane"
}